{
  "gene_name": "DENN domain-containing protein 2A",
  "gene": "UniProtKB:Q9ULE3",
  "gene_symbol": "DENND2A",
  "term_label": "actin cytoskeleton",
  "term_id": "GO:0015629"
}